neuron remodeling [GO:0016322] (biological process) Relationships: is a type of neuron maturation [GO:0042551] Definition: The developmentally regulated remodeling of neuronal projections such as pruning to eliminate the extra dendrites and axons projections set up in early stages of nervous system development. Regulation: regulated by regulation of neuron remodeling [GO:1904799]; negatively regulated by negative regulation of neuron remodeling [GO:1904800]; positively regulated by positive regulation of neuron remodeling [GO:1904801] Sources: GOC:hb Also known as: neuron remodelling, neuronal remodeling, axon pruning